{
  "term_label": "apoptotic process",
  "gene_symbol": "AIFM1",
  "gene_name": "Apoptosis-inducing factor 1, mitochondrial",
  "term_id": "GO:0006915",
  "gene": "UniProtKB:O95831"
}